{
  "gene": "UniProtKB:Q8N3C0",
  "term_id": "UNKNOWN:0002",
  "gene_symbol": "ASCC3",
  "term_label": "Unknown biological process",
  "gene_name": "Activating signal cointegrator 1 complex subunit 3"
}